{
  "term_id": "GO:0004888",
  "term_label": "transmembrane signaling receptor activity",
  "gene_symbol": "SORL1",
  "gene_name": "Sortilin-related receptor",
  "gene": "UniProtKB:Q92673"
}